{
  "term_id": "GO:0005549",
  "gene_symbol": "OR5AN1",
  "gene": "UniProtKB:Q8NGI8",
  "term_label": "odorant binding",
  "gene_name": "Olfactory receptor 5AN1"
}